{
  "term_id": "GO:0015645",
  "gene_name": "Acyl-coenzyme A synthetase ACSM6, mitochondrial",
  "term_label": "fatty acid ligase activity",
  "gene_symbol": "ACSM6",
  "gene": "UniProtKB:Q6P461"
}